{
  "term_label": "olfactory receptor activity",
  "gene_name": "Olfactory receptor 4M2",
  "term_id": "GO:0004984",
  "gene_symbol": "OR4M2B",
  "gene": "UniProtKB:A0A0X1KG70"
}